regulation of termination of DNA-templated transcription [GO:0031554] (biological process) Sources: GOC:mlg, GOC:txnOH Subtypes: GO:0060566, negative regulation of termination of DNA-templated transcription [GO:0060567], GO:1904594, regulation of termination of RNA polymerase I transcription [GO:2000730] Also known as: regulation of DNA-dependent transcription, termination, regulation of DNA-templated transcription, termination, regulation of transcription termination, DNA-dependent, transcription antiterminator activity Relationships: is a type of regulation of protein-containing complex disassembly [GO:0043244]; is a type of regulation of RNA biosynthetic process [GO:2001141]; regulates DNA-templated transcription termination [GO:0006353] Definition: Any process that modulates the frequency, rate, extent, or location of DNA-templated transcription termination, the process in which transcription is completed; the formation of phosphodiester bonds ceases, the RNA-DNA hybrid dissociates, and RNA polymerase releases the DNA.